{
  "gene": "UniProtKB:P0C2L3",
  "gene_name": "Protein FAM163B",
  "gene_symbol": "FAM163B",
  "term_id": "UNKNOWN:0001",
  "term_label": "Unknown molecular function"
}